{
  "term_id": "UNKNOWN:0002",
  "gene_name": "T cell receptor alpha joining 13 (Fragment)",
  "gene": "UniProtKB:A0A075B709",
  "term_label": "Unknown biological process",
  "gene_symbol": "TRAJ13"
}